{
  "term_id": "GO:0070830",
  "gene": "UniProtKB:P56747",
  "term_label": "bicellular tight junction assembly",
  "gene_name": "Claudin-6",
  "gene_symbol": "CLDN6"
}